transcription factor TFIIK complex [GO:0070985] (cellular component) Relationships: is_a GO:0090575; BFO_0000050 transcription factor TFIIH holo complex [GO:0005675] Definition: A transcription factor complex that forms part of the holo TFIIH complex. In Saccharomyces/human, TFIIK contains Ccl1p/Cyclin H, Tfb3p/MAT1 and Kin28p/CDK7. Also known as: TFIIK complex, Mcs6/Mcs2/Pmh1 complex, cyclin H-CDK7 complex References: PMID:19818408, PMID:22572993 Sources: GOC:mah